{
  "gene_name": "Putative uncharacterized protein FLJ45256",
  "term_id": "UNKNOWN:0002",
  "gene_symbol": "Q6ZSR6",
  "gene": "UniProtKB:Q6ZSR6",
  "term_label": "Unknown biological process"
}